{
  "gene": "UniProtKB:Q8IWV2",
  "term_id": "GO:0098632",
  "gene_symbol": "CNTN4",
  "gene_name": "Contactin-4",
  "term_label": "cell-cell adhesion mediator activity"
}